cell migration involved in mammary placode formation [GO:0060619] (biological process) Definition: The orderly movement of epithelial cells within the mammary line that contributes to the formation of the mammary placode. References: PMID:12558599 Sources: GOC:dph Relationships: is a type of epithelial cell migration [GO:0010631]; is part of mammary placode formation [GO:0060596]